{
  "gene_symbol": "C2CD3",
  "term_label": "centriole elongation",
  "term_id": "GO:0061511",
  "gene": "UniProtKB:Q4AC94",
  "gene_name": "C2 domain-containing protein 3"
}